{
  "gene_symbol": "CLDN1",
  "term_id": "GO:0016338",
  "gene_name": "Claudin-1",
  "gene": "UniProtKB:O95832",
  "term_label": "calcium-independent cell-cell adhesion"
}